{
  "term_label": "keratinization",
  "gene": "UniProtKB:Q14CN4",
  "gene_symbol": "KRT72",
  "term_id": "GO:0031424",
  "gene_name": "Keratin, type II cytoskeletal 72"
}